{
  "gene": "UniProtKB:Q96M93",
  "gene_symbol": "ADAD1",
  "term_label": "RNA processing",
  "term_id": "GO:0006396",
  "gene_name": "Adenosine deaminase domain-containing protein 1"
}